{
  "term_label": "Unknown cellular component",
  "gene_symbol": "LEKR1",
  "gene": "UniProtKB:Q6ZMV7",
  "term_id": "UNKNOWN:0003",
  "gene_name": "Protein LEKR1"
}